{
  "gene": "UniProtKB:Q9NRI5",
  "gene_symbol": "DISC1",
  "gene_name": "Disrupted in schizophrenia 1 protein",
  "term_label": "molecular adaptor activity",
  "term_id": "GO:0060090"
}